{
  "term_label": "P-body",
  "term_id": "GO:0000932",
  "gene_name": "Trinucleotide repeat-containing gene 6B protein",
  "gene_symbol": "TNRC6B",
  "gene": "UniProtKB:Q9UPQ9"
}